{
  "gene_symbol": "FOXS1",
  "gene": "UniProtKB:O43638",
  "gene_name": "Forkhead box protein S1",
  "term_id": "GO:0030154",
  "term_label": "cell differentiation"
}